{
  "gene_symbol": "EIF2S1",
  "term_id": "GO:0005850",
  "term_label": "eukaryotic translation initiation factor 2 complex",
  "gene_name": "Eukaryotic translation initiation factor 2 subunit 1",
  "gene": "UniProtKB:P05198"
}